protein-containing complex disassembly [GO:0032984] (BP) Relationships: is a type of cellular component disassembly [GO:0022411]; is a type of GO:0043933 Definition: The disaggregation of a protein-containing macromolecular complex into its constituent components. Also known as: protein complex disassembly, cellular macromolecule complex disassembly, cellular protein complex disassembly, macromolecule complex disassembly Subtypes: protein-DNA-RNA complex disassembly [GO:0001117], translational termination [GO:0006415], myosin filament disassembly [GO:0031035], protein-carbohydrate complex disassembly [GO:0032985], protein-DNA complex disassembly [GO:0032986], protein-lipid complex disassembly [GO:0032987], protein-RNA complex disassembly [GO:0032988], SNARE complex disassembly [GO:0035494], GO:0044721, protein depolymerization [GO:0051261], autophagosome maturation [GO:0097352], mitotic nuclear pore complex disassembly [GO:0140516], proteasome complex disassembly [GO:1903009], exon-exon junction complex disassembly [GO:1903259], chaperone-mediated autophagy translocation complex disassembly [GO:1904764], beta-catenin destruction complex disassembly [GO:1904886], ESCRT complex disassembly [GO:1904896], TORC2 complex disassembly [GO:1905670], SCF complex disassembly in response to cadmium stress [GO:1990171] Regulation: negatively regulated by negative regulation of protein-containing complex disassembly [GO:0043242]; positively regulated by positive regulation of protein-containing complex disassembly [GO:0043243]; regulated by regulation of protein-containing complex disassembly [GO:0043244] Sources: GOC:mah